{
  "gene_name": "Histone H1.3",
  "gene": "UniProtKB:P16402",
  "term_label": "negative regulation of DNA recombination",
  "term_id": "GO:0045910",
  "gene_symbol": "H1-3"
}